{
  "gene_symbol": "USP43",
  "gene": "UniProtKB:Q70EL4",
  "gene_name": "Ubiquitin carboxyl-terminal hydrolase 43",
  "term_label": "Unknown cellular component",
  "term_id": "UNKNOWN:0003"
}